{
  "term_id": "GO:1990904",
  "term_label": "ribonucleoprotein complex",
  "gene_name": "Elongation factor 2",
  "gene": "UniProtKB:P13639",
  "gene_symbol": "EEF2"
}